{
  "gene": "UniProtKB:Q9HB66",
  "gene_name": "Alternative protein MKKS",
  "gene_symbol": "MKKS",
  "term_label": "Unknown molecular function",
  "term_id": "UNKNOWN:0001"
}